{
  "term_id": "GO:0004620",
  "gene": "UniProtKB:Q9Y6Y8",
  "gene_name": "SEC23-interacting protein",
  "gene_symbol": "SEC23IP",
  "term_label": "phospholipase activity"
}